HUSH complex [GO:0140283] (cellular component) Relationships: is a type of chromatin silencing complex [GO:0005677] References: PMID:39013473, PMID:39489739 Definition: A protein complex that mediates transcriptional silencing of mobile genetic elements, such as retroviruses and transposable elements. In human, it is composed of TASOR, PPHLN1 and MPHOSPH8.